{
  "gene": "UniProtKB:Q8NGZ2",
  "term_id": "UNKNOWN:0003",
  "gene_symbol": "OR14K1",
  "term_label": "Unknown cellular component",
  "gene_name": "Olfactory receptor 14K1"
}